{
  "gene_name": "Meiosis 1 arrest protein",
  "term_id": "UNKNOWN:0001",
  "term_label": "Unknown molecular function",
  "gene": "UniProtKB:Q8TC57",
  "gene_symbol": "M1AP"
}